positive regulation of sevenless signaling pathway [GO:0045874] (BP) Definition: Any process that activates or increases the frequency, rate or extent of the sevenless signaling pathway. Relationships: is a type of GO:0009967; is_a regulation of sevenless signaling pathway [GO:0045501]; positively regulates sevenless signaling pathway [GO:0045500] Also known as: positive regulation of sev signaling pathway, positive regulation of sevenless signalling pathway, up regulation of sevenless signaling pathway, up-regulation of sevenless signaling pathway, upregulation of sevenless signaling pathway, activation of sevenless signaling pathway, stimulation of sevenless signaling pathway Sources: GOC:go_curators